{
  "term_label": "response to peptide hormone",
  "gene_name": "Signal transducer and activator of transcription 5B",
  "gene_symbol": "STAT5B",
  "term_id": "GO:0043434",
  "gene": "UniProtKB:P51692"
}